{
  "gene_symbol": "HLA-DQA2",
  "term_id": "GO:0002503",
  "gene": "UniProtKB:P01906",
  "term_label": "peptide antigen assembly with MHC class II protein complex",
  "gene_name": "HLA class II histocompatibility antigen, DQ alpha 2 chain"
}